{
  "gene": "UniProtKB:Q6P4H8",
  "gene_symbol": "ATPSCKMT",
  "gene_name": "ATP synthase subunit C lysine N-methyltransferase",
  "term_id": "GO:0016279",
  "term_label": "protein-lysine N-methyltransferase activity"
}